{
  "gene": "UniProtKB:Q13426",
  "term_label": "DNA-dependent protein kinase-DNA ligase 4 complex",
  "gene_symbol": "XRCC4",
  "gene_name": "DNA repair protein XRCC4",
  "term_id": "GO:0005958"
}